{
  "gene_name": "Kelch-like protein 35",
  "gene_symbol": "KLHL35",
  "term_id": "GO:1990756",
  "gene": "UniProtKB:Q6PF15",
  "term_label": "ubiquitin-like ligase-substrate adaptor activity"
}